{
  "term_id": "UNKNOWN:0002",
  "gene": "UniProtKB:Q86VU5",
  "term_label": "Unknown biological process",
  "gene_name": "Catechol O-methyltransferase domain-containing protein 1",
  "gene_symbol": "COMTD1"
}